{
  "term_label": "negative regulation of growth hormone receptor signaling pathway",
  "gene_symbol": "LEPROTL1",
  "term_id": "GO:0060400",
  "gene_name": "Leptin receptor overlapping transcript-like 1",
  "gene": "UniProtKB:O95214"
}